{
  "term_id": "GO:0050435",
  "gene_name": "Insulin-degrading enzyme",
  "term_label": "amyloid-beta metabolic process",
  "gene": "UniProtKB:P14735",
  "gene_symbol": "IDE"
}